{
  "gene": "UniProtKB:Q9H082",
  "term_label": "GTP binding",
  "gene_name": "Ras-related protein Rab-33B",
  "term_id": "GO:0005525",
  "gene_symbol": "RAB33B"
}